male sex determination [GO:0030238] (biological process) Definition: The specification of male sex of an individual organism. Sources: GOC:mah Subtypes: male germ-line sex determination [GO:0019100], male somatic sex determination [GO:0019102] Relationships: is a type of sex determination [GO:0007530]; is part of multicellular organism development [GO:0007275]